isohexenylglutaconyl-CoA hydratase activity [GO:0050005] (molecular function) Sources: EC:4.2.1.57, RHEA:24144 Relationships: is a type of hydro-lyase activity [GO:0016836] Definition: Catalysis of the reaction: 3-hydroxy-3-(4-methylpent-3-en-1-yl)glutaryl-CoA = 3-(4-methylpent-3-en-1-yl)pent-2-enedioyl-CoA + H2O. Also known as: 3-hydroxy-3-(4-methylpent-3-en-1-yl)glutaryl-CoA hydro-lyase [3-(4-methylpent-3-en-1-yl)pent-2-enedioyl-CoA-forming], 3-hydroxy-3-(4-methylpent-3-en-1-yl)glutaryl-CoA hydro-lyase activity, 3-hydroxy-3-isohexenylglutaryl-CoA-hydrolase activity, beta-isohexenylglutaconyl-CoA-hydratase activity, isohexenylglutaconyl coenzyme A hydratase activity